{
  "term_label": "lipid droplet",
  "term_id": "GO:0005811",
  "gene": "UniProtKB:Q9Y5L2",
  "gene_symbol": "HILPDA",
  "gene_name": "Hypoxia-inducible lipid droplet-associated protein"
}